{
  "gene": "UniProtKB:Q9HB63",
  "term_label": "substrate adhesion-dependent cell spreading",
  "term_id": "GO:0034446",
  "gene_name": "Netrin-4",
  "gene_symbol": "NTN4"
}